{
  "term_label": "extracellular space",
  "gene_symbol": "CCN4",
  "term_id": "GO:0005615",
  "gene": "UniProtKB:O95388",
  "gene_name": "CCN family member 4"
}